B cell tolerance induction in mucosal-associated lymphoid tissue [GO:0002402] (biological process) Sources: GOC:jal, ISBN:0781735149 Definition: Tolerance induction taking place in the mucosal-associated lymphoid tissue (MALT) mediated by B cells. Also known as: B cell tolerance induction in MALT Relationships: is a type of tolerance induction in mucosal-associated lymphoid tissue [GO:0002401]; is a type of peripheral B cell tolerance induction [GO:0002451]